{
  "gene_symbol": "NUBPL",
  "gene": "UniProtKB:Q8TB37",
  "term_label": "iron-sulfur cluster assembly",
  "term_id": "GO:0016226",
  "gene_name": "Iron-sulfur protein NUBPL"
}